{
  "term_label": "retrograde vesicle-mediated transport, Golgi to endoplasmic reticulum",
  "term_id": "GO:0006890",
  "gene": "UniProtKB:Q969X5",
  "gene_name": "Endoplasmic reticulum-Golgi intermediate compartment protein 1",
  "gene_symbol": "ERGIC1"
}